phosphatidylcholine-retinol O-acyltransferase activity [GO:0047173] (molecular function) Definition: Catalysis of the reaction: a 1,2-diacyl-sn-glycero-3-phosphocholine + all-trans-retinol--[retinol-binding protein] = a 2-acyl-sn-glycero-3-phosphocholine + an all-trans-retinyl ester + apo--[retinol-binding protein]. Recognizes the substrate both in free form and when bound to cellular-retinol-binding-protein, but has higher affinity for the bound form. Sources: RHEA:17469 Also known as: lecithin--retinol acyltransferase activity, phosphatidylcholine:retinol-(cellular-retinol-binding-protein) O-acyltransferase activity, phosphatidylcholine:retinol-[cellular-retinol-binding-protein] O-acyltransferase activity Relationships: is a type of O-acyltransferase activity [GO:0008374]